{
  "gene": "UniProtKB:P09228",
  "term_label": "vesicle",
  "gene_symbol": "CST2",
  "term_id": "GO:0031982",
  "gene_name": "Cystatin-SA"
}